endocardial cushion cell differentiation [GO:0061443] (biological process) Regulation: regulated by regulation of endocardial cushion cell differentiation [GO:0120074]; positively regulated by positive regulation of endocardial cushion cell differentiation [GO:0120075]; negatively regulated by negative regulation of endocardial cushion cell differentiation [GO:0120076] Definition: The process in which a relatively unspecialized cell acquires the specialized structural and/or functional features of an endocardial cushion cell. Relationships: is_a cardiocyte differentiation [GO:0035051]; is part of GO:0003197 Sources: GOC:BHF, GOC:dph